{
  "gene": "UniProtKB:O95718",
  "gene_symbol": "ESRRB",
  "gene_name": "Steroid hormone receptor ERR2",
  "term_id": "GO:0000785",
  "term_label": "chromatin"
}